{
  "term_id": "GO:0007186",
  "gene": "UniProtKB:Q9UHX3",
  "gene_name": "Adhesion G protein-coupled receptor E2",
  "gene_symbol": "ADGRE2",
  "term_label": "G protein-coupled receptor signaling pathway"
}